{
  "gene_name": "Insulin receptor-related protein",
  "gene_symbol": "INSRR",
  "term_label": "insulin receptor complex",
  "gene": "UniProtKB:P14616",
  "term_id": "GO:0005899"
}